{
  "gene": "UniProtKB:P09105",
  "term_label": "hemoglobin complex",
  "gene_symbol": "HBQ1",
  "gene_name": "Hemoglobin subunit theta-1",
  "term_id": "GO:0005833"
}